granulosa cell proliferation [GO:1990739] (BP) Relationships: is a type of epithelial cell proliferation [GO:0050673] References: PMID:22383759 Regulation: regulated by GO:1904195; negatively regulated by GO:1904196; RO_0002213 by positive regulation of granulosa cell proliferation [GO:1904197] Definition: The multiplication or reproduction of granulosa cells, resulting in the expansion of the granulosa cells population. A granulosa cell is a supporting cell for the developing female gamete in the ovary of mammals. They develop from the coelomic epithelial cells of the gonadal ridge.